{
  "term_id": "GO:0050830",
  "term_label": "defense response to Gram-positive bacterium",
  "gene_name": "Defensin-6",
  "gene": "UniProtKB:Q01524",
  "gene_symbol": "DEFA6"
}